{
  "term_label": "exocytosis",
  "gene_symbol": "RAB8A",
  "gene_name": "Ras-related protein Rab-8A",
  "term_id": "GO:0006887",
  "gene": "UniProtKB:P61006"
}